alpha-N-acetylglucosaminidase activity [GO:0004561] (molecular function) Relationships: is a type of hexosaminidase activity [GO:0015929] Also known as: N-acetyl-alpha-D-glucosaminidase activity, N-acetyl-alpha-glucosaminidase activity, NAG activity, alpha-D-2-acetamido-2-deoxyglucosidase activity, alpha-N-acetyl-D-glucosaminide N-acetylglucosaminohydrolase activity, alpha-acetylglucosaminidase activity Definition: Catalysis of the hydrolysis of terminal non-reducing N-acetyl-D-glucosamine residues in N-acetyl-alpha-D-glucosaminides. Sources: EC:3.2.1.50